mannan synthase activity [GO:0051753] (molecular function) Definition: Catalysis of the reaction: mannan(n) + GDP-mannose = mannan(n+1) + GDP. This reaction is the formation of the beta-(1->4)-linked mannan backbone in substrates such as galactomannan. Relationships: is a type of beta-1,4-mannosyltransferase activity [GO:0019187] Also known as: mannan beta-1,4-mannosyltransferase activity, galactomannan beta-1,4-mannosyltransferase activity References: PMID:14726589